dolichol kinase activity [GO:0004168] (molecular function) Relationships: is a type of kinase activity [GO:0016301]; is_a phosphotransferase activity, alcohol group as acceptor [GO:0016773] Also known as: CTP:dolichol O-phosphotransferase activity, dolichol phosphokinase activity Definition: Catalysis of the reaction: CTP + dolichol = CDP + dolichyl phosphate. Sources: EC:2.7.1.108